{
  "gene_name": "Disintegrin and metalloproteinase domain-containing protein 29",
  "gene_symbol": "ADAM29",
  "gene": "UniProtKB:Q9UKF5",
  "term_id": "GO:0008584",
  "term_label": "male gonad development"
}